positive regulation of xanthophore differentiation [GO:0050946] (BP) Definition: Any process that activates or increases the frequency, rate or extent of xanthophore differentiation. Sources: GOC:ai Also known as: up regulation of xanthophore differentiation, up-regulation of xanthophore differentiation, upregulation of xanthophore differentiation, activation of xanthophore differentiation, stimulation of xanthophore differentiation Note: Note that this term refers to xanthophores in the sense of specialized pigment-producing cells, and should not be confused with the cellular component term 'xanthophore ; GO:0031633', which refers to a subcellular structure. Relationships: is a type of regulation of xanthophore differentiation [GO:0050938]; is a type of positive regulation of pigment cell differentiation [GO:0050942]; positively regulates GO:0050936